{
  "gene_symbol": "AKAP1",
  "gene_name": "A-kinase anchor protein 1, mitochondrial",
  "gene": "UniProtKB:Q92667",
  "term_id": "GO:0005739",
  "term_label": "mitochondrion"
}